{
  "gene_symbol": "OR8D2",
  "gene_name": "Olfactory receptor 8D2",
  "gene": "UniProtKB:Q9GZM6",
  "term_label": "Unknown cellular component",
  "term_id": "UNKNOWN:0003"
}